{
  "term_id": "GO:0006182",
  "gene_name": "Guanylate cyclase soluble subunit alpha-1",
  "gene": "UniProtKB:Q02108",
  "term_label": "cGMP biosynthetic process",
  "gene_symbol": "GUCY1A1"
}